phytochelatin 3 import into vacuole [GO:0036247] (biological process) References: PMID:19001374 Sources: GOC:al Also known as: PC3 import into vacuole Definition: The directed movement of phytochelatin 3 (PC3) into the vacuole. Phytochelatin 3 is a glutathione-related peptide composed of (gamma-Glu-Cys)n-Gly where n=3, and where the Glu and Cys residues are linked through a gamma-carboxylamide bond. Relationships: is a type of oligopeptide transmembrane transport [GO:0035672]; is a type of phytochelatin import into vacuole [GO:0071995]